dinoflagellate epicone [GO:0097613] (CC) Definition: The part of a dinoflagellate cell above the cingulum; also referred to as the anterior portion of a dinoflagellate cell. It is separated from the hypocone by the cingulum. Also known as: epicone, episome, epitheca Relationships: is a type of GO:0110165 Sources: GOC:at, Wikipedia:Dinoflagellate#Morphology, http://tolweb.org/Dinoflagellates/2445 Note: The term name refers to a taxonomic group to make the label unique with respect to similarly-named anatomical structures.